{
  "gene_symbol": "NDUFB4",
  "term_label": "Unknown molecular function",
  "gene_name": "NADH dehydrogenase [ubiquinone] 1 beta subcomplex subunit 4",
  "gene": "UniProtKB:O95168",
  "term_id": "UNKNOWN:0001"
}